retinol binding [GO:0019841] (molecular function) Relationships: is a type of retinoid binding [GO:0005501]; is a type of vitamin binding [GO:0019842]; is a type of GO:0043178 Also known as: vitamin A1 alcohol binding, vitamin A1 binding Sources: GOC:curators Definition: Binding to retinol, vitamin A1, 2,6,6-trimethyl-1-(9'-hydroxy-3',7'-dimethylnona-1',3',5',7'-tetraenyl)cyclohex-1-ene, one of the three components that makes up vitamin A. Retinol is an intermediate in the vision cycle and it also plays a role in growth and differentiation. Subtypes: GO:1904768